{
  "gene_symbol": "ERF",
  "term_label": "cell differentiation",
  "gene": "UniProtKB:P50548",
  "term_id": "GO:0030154",
  "gene_name": "ETS domain-containing transcription factor ERF"
}